{
  "term_label": "Unknown biological process",
  "gene_symbol": "TTC28",
  "gene": "UniProtKB:Q96AY4",
  "term_id": "UNKNOWN:0002",
  "gene_name": "Tetratricopeptide repeat protein 28"
}